{
  "term_label": "regulation of G1/S transition of mitotic cell cycle",
  "gene": "UniProtKB:P42771",
  "gene_name": "Cyclin-dependent kinase inhibitor 2A",
  "gene_symbol": "CDKN2A",
  "term_id": "GO:2000045"
}